{
  "gene_symbol": "PNPO",
  "gene": "UniProtKB:Q9NVS9",
  "term_label": "pyridoxal phosphate biosynthetic process",
  "gene_name": "Pyridoxine-5'-phosphate oxidase",
  "term_id": "GO:0042823"
}